{
  "term_label": "cytoplasm",
  "gene": "UniProtKB:Q9HC16",
  "gene_symbol": "APOBEC3G",
  "gene_name": "DNA dC-dU-editing enzyme APOBEC-3G",
  "term_id": "GO:0005737"
}